{
  "term_id": "GO:0016020",
  "gene_name": "Rho GDP-dissociation inhibitor 1",
  "gene_symbol": "ARHGDIA",
  "term_label": "membrane",
  "gene": "UniProtKB:P52565"
}